regulation of erythrophore differentiation [GO:0048778] (biological process) Sources: GOC:mh Relationships: is a type of GO:0050932; RO_0002211 erythrophore differentiation [GO:0048773] Definition: Any process that modulates the frequency, rate or extent of erythrophore differentiation. Subtypes: GO:0048779, positive regulation of erythrophore differentiation [GO:0048780]